{
  "gene_name": "Aminopeptidase NAALADL1",
  "gene_symbol": "NAALADL1",
  "term_label": "Unknown cellular component",
  "term_id": "UNKNOWN:0003",
  "gene": "UniProtKB:Q9UQQ1"
}